{
  "term_id": "GO:0022900",
  "gene_symbol": "FDX2",
  "gene": "UniProtKB:Q6P4F2",
  "gene_name": "Ferredoxin-2, mitochondrial",
  "term_label": "electron transport chain"
}